{
  "gene_symbol": "POLR2M",
  "gene_name": "DNA-directed RNA polymerase II subunit GRINL1A",
  "term_label": "Unknown molecular function",
  "gene": "UniProtKB:P0CAP2",
  "term_id": "UNKNOWN:0001"
}